{
  "gene_name": "Interleukin-9",
  "term_id": "GO:0005140",
  "gene_symbol": "IL9",
  "term_label": "interleukin-9 receptor binding",
  "gene": "UniProtKB:P15248"
}